thiocyanate hydrolase activity [GO:0018760] (molecular function) Definition: Catalysis of the reaction: H2O + 2 H+ + thiocyanate = carbonyl sulfide + NH4. Sources: EC:3.5.5.8, RHEA:21464 Also known as: thiocyanate aminohydrolase activity Relationships: is a type of hydrolase activity, acting on carbon-nitrogen (but not peptide) bonds, in nitriles [GO:0016815]